{
  "gene_symbol": "KRTAP19-5",
  "term_id": "UNKNOWN:0002",
  "gene": "UniProtKB:Q3LI72",
  "term_label": "Unknown biological process",
  "gene_name": "Keratin-associated protein 19-5"
}